3-dehydro-L-gulonate 2-dehydrogenase activity [GO:0047559] (molecular function) Sources: EC:1.1.1.130, MetaCyc:3-DEHYDRO-L-GULONATE-2-DEHYDROGENASE-RXN Also known as: 2,3-diketo-L-gulonate reductase activity, 3-dehydro-L-gulonate:NAD(P)+ 2-oxidoreductase activity, 3-keto-L-gulonate dehydrogenase activity, 3-ketogulonate dehydrogenase activity Definition: Catalysis of the reaction: 3-dehydro-L-gulonate + NAD(P)+ = (4R,5S)-4,5,6-trihydroxy-2,3-dioxohexanoate + NAD(P)H + H+. Relationships: is a type of oxidoreductase activity, acting on the CH-OH group of donors, NAD or NADP as acceptor [GO:0016616]